{
  "term_id": "UNKNOWN:0003",
  "term_label": "Unknown cellular component",
  "gene_symbol": "STPG1",
  "gene": "UniProtKB:Q5TH74",
  "gene_name": "O(6)-methylguanine-induced apoptosis 2"
}